negative regulation of circadian sleep/wake cycle, wakefulness [GO:1904326] (biological process) References: PMID:10923657 Sources: GOC:TermGenie, GO_REF:0000058 Definition: Any process that stops, prevents or reduces the frequency, rate or extent of circadian sleep/wake cycle, wakefulness. Relationships: is a type of regulation of circadian sleep/wake cycle, wakefulness [GO:0010840]; is_a GO:0042754; is a type of negative regulation of behavior [GO:0048521]; negatively regulates GO:0042746 Also known as: down regulation of circadian sleep/wake cycle, wakefulness, down-regulation of circadian sleep/wake cycle, wakefulness, downregulation of circadian sleep/wake cycle, wakefulness, inhibition of circadian sleep/wake cycle, wakefulness